{
  "gene_name": "Protein phosphatase 1 regulatory subunit 17",
  "term_label": "Unknown cellular component",
  "gene_symbol": "PPP1R17",
  "term_id": "UNKNOWN:0003",
  "gene": "UniProtKB:O96001"
}